{
  "term_label": "histone deacetylase binding",
  "gene": "UniProtKB:Q5PSV4",
  "term_id": "GO:0042826",
  "gene_name": "Breast cancer metastasis-suppressor 1-like protein",
  "gene_symbol": "BRMS1L"
}